{
  "term_label": "ribosome biogenesis",
  "gene": "UniProtKB:Q9BQ67",
  "gene_name": "Glutamate-rich WD repeat-containing protein 1",
  "term_id": "GO:0042254",
  "gene_symbol": "GRWD1"
}